{
  "gene_symbol": "EPGN",
  "term_label": "epidermal growth factor receptor signaling pathway",
  "gene_name": "Epigen",
  "gene": "UniProtKB:Q6UW88",
  "term_id": "GO:0007173"
}